{
  "term_id": "GO:0045892",
  "gene_symbol": "ZNF541",
  "gene": "UniProtKB:Q9H0D2",
  "term_label": "negative regulation of DNA-templated transcription",
  "gene_name": "Zinc finger protein 541"
}